{
  "term_label": "Unknown biological process",
  "gene_name": "Protein GDF5-AS1, mitochondrial",
  "gene_symbol": "GDF5-AS1",
  "term_id": "UNKNOWN:0002",
  "gene": "UniProtKB:Q5U4N7"
}